cellular response to high density lipoprotein particle stimulus [GO:0071403] (biological process) Sources: GOC:mah Relationships: is a type of cellular response to lipoprotein particle stimulus [GO:0071402] Also known as: response to high density lipoprotein particle, response to high density lipoprotein particle stimulus, cellular response to high-density lipoprotein particle stimulus Definition: Any process that results in a change in state or activity of a cell (in terms of movement, secretion, enzyme production, gene expression, etc.) as a result of a high density lipoprotein particle stimulus.